{
  "gene_symbol": "THRB",
  "term_id": "GO:0004879",
  "gene": "UniProtKB:P10828",
  "term_label": "nuclear receptor activity",
  "gene_name": "Thyroid hormone receptor beta"
}